{
  "gene": "UniProtKB:Q96JG8",
  "gene_name": "Melanoma-associated antigen D4",
  "term_label": "negative regulation of transcription by RNA polymerase II",
  "gene_symbol": "MAGED4",
  "term_id": "GO:0000122"
}